{
  "term_label": "Unknown biological process",
  "gene_symbol": "C1orf94",
  "term_id": "UNKNOWN:0002",
  "gene": "UniProtKB:Q6P1W5",
  "gene_name": "Uncharacterized protein C1orf94"
}